{
  "term_id": "GO:0008970",
  "gene_name": "Phospholipase A and acyltransferase 2",
  "gene": "UniProtKB:Q9NWW9",
  "term_label": "phospholipase A1 activity",
  "gene_symbol": "PLAAT2"
}